{
  "gene_name": "17-beta-hydroxysteroid dehydrogenase 13",
  "term_id": "GO:0016616",
  "gene_symbol": "HSD17B13",
  "term_label": "oxidoreductase activity, acting on the CH-OH group of donors, NAD or NADP as acceptor",
  "gene": "UniProtKB:Q7Z5P4"
}